negative regulation of DNA replication [GO:0008156] (biological process) Relationships: is a type of regulation of DNA replication [GO:0006275]; is a type of negative regulation of DNA metabolic process [GO:0051053]; negatively regulates GO:0006260 Definition: Any process that stops, prevents, or reduces the frequency, rate or extent of DNA replication. Subtypes: GO:2000104 Also known as: down regulation of DNA replication, down-regulation of DNA replication, downregulation of DNA replication, inhibition of DNA replication, DNA replication inhibitor Sources: GOC:go_curators